symbiont-mediated perturbation of host G protein-coupled receptor signal transduction pathway [GO:0075118] (biological process) Sources: GOC:pamgo_curators Definition: A process by which a symbiont alters or subverts the normal execution of a host G protein-coupled receptor signal transduction pathway. The host is defined as the larger of the organisms involved in a symbiotic interaction. Subtypes: GO:0075120, symbiont-mediated activation of host G protein-coupled receptor signal transduction [GO:0141104] Relationships: is a type of GO:0075109 Also known as: modulation by symbiont of host G protein-coupled receptor signal transduction, modulation by symbiont of host G-protein coupled receptor protein signal transduction, perturbation of host G protein-coupled receptor signal transduction pathway, modulation by symbiont of host signal transduction mediated by G-protein alpha subunit, modulation by symbiont of host signal transduction mediated by G-protein beta subunit, modulation by symbiont of host signal transduction mediated by G-protein gamma subunit